positive regulation of fructose 1,6-bisphosphate metabolic process [GO:0060552] (biological process) Definition: Any process that increases the rate, frequency or extent of fructose 1,6-bisphosphate metabolism. Fructose 1,6-bisphosphate metabolism is the chemical reactions and pathways involving fructose 1,6-bisphosphate, also known as FBP. The D enantiomer is a metabolic intermediate in glycolysis and gluconeogenesis. Sources: GOC:BHF, GOC:dph, GOC:tb Relationships: is_a positive regulation of phosphate metabolic process [GO:0045937]; positively regulates GO:0030388